{
  "term_id": "GO:0005634",
  "term_label": "nucleus",
  "gene": "UniProtKB:P10909",
  "gene_name": "Clusterin",
  "gene_symbol": "CLU"
}